{
  "gene": "UniProtKB:Q92793",
  "gene_symbol": "CREBBP",
  "term_id": "GO:0004402",
  "term_label": "histone acetyltransferase activity",
  "gene_name": "CREB-binding protein"
}